{
  "term_label": "axon",
  "gene": "UniProtKB:Q02246",
  "term_id": "GO:0030424",
  "gene_symbol": "CNTN2",
  "gene_name": "Contactin-2"
}